{
  "gene_symbol": "YWHAG",
  "gene_name": "14-3-3 protein gamma",
  "term_label": "protein kinase C binding",
  "term_id": "GO:0005080",
  "gene": "UniProtKB:P61981"
}